magnesium ion transmembrane transporter activity [GO:0015095] (molecular function) Relationships: is a type of GO:0046873; is part of magnesium ion transmembrane transport [GO:1903830] Sources: GOC:dgf Subtypes: GO:0015444, magnesium:sodium antiporter activity [GO:0061768] Definition: Enables the transfer of magnesium (Mg) ions from one side of a membrane to the other.